pyrrole-2-carboxylate monooxygenase (NADH) activity [GO:0034938] (molecular function) Definition: Catalysis of the reaction: H+ + NADH + O2 + pyrrole-2-carboxylate = 5-hydroxypyrrole-2-carboxylate + H2O + NAD+. Sources: RHEA:30351 Relationships: is a type of oxidoreductase activity, acting on paired donors, with incorporation or reduction of molecular oxygen, NAD(P)H as one donor, and incorporation of one atom of oxygen [GO:0016709]